{
  "term_id": "GO:0007032",
  "gene_symbol": "ANXA8",
  "gene_name": "Annexin A8",
  "term_label": "endosome organization",
  "gene": "UniProtKB:P13928"
}